dopamine neurotransmitter receptor activity, coupled via Gs [GO:0001588] (molecular function) Relationships: is a type of GO:0004952 Also known as: dopamine D1 receptor activity, dopamine D5 receptor activity Sources: GOC:mah, ISBN:0953351033, IUPHAR_RECEPTOR:2252, IUPHAR_RECEPTOR:2260 Definition: Combining with the neurotransmitter dopamine and activating adenylate cyclase via coupling to Gs to initiate a change in cell activity.